{
  "gene_symbol": "KATNA1",
  "term_id": "GO:0016887",
  "gene_name": "Katanin p60 ATPase-containing subunit A1",
  "gene": "UniProtKB:O75449",
  "term_label": "ATP hydrolysis activity"
}